{
  "term_id": "GO:0036126",
  "gene_symbol": "TCP11",
  "gene_name": "T-complex protein 11 homolog",
  "term_label": "sperm flagellum",
  "gene": "UniProtKB:Q8WWU5"
}